{
  "term_label": "axon",
  "term_id": "GO:0030424",
  "gene": "UniProtKB:P14616",
  "gene_symbol": "INSRR",
  "gene_name": "Insulin receptor-related protein"
}